nucleoside triphosphate catabolic process [GO:0009143] (biological process) Definition: The chemical reactions and pathways resulting in the breakdown of a nucleoside triphosphate, a compound consisting of a nucleobase linked to a deoxyribose or ribose sugar esterified with triphosphate on the sugar. Sources: GOC:go_curators, ISBN:0198506732 Relationships: is a type of nucleoside triphosphate metabolic process [GO:0009141]; is a type of nucleoside phosphate catabolic process [GO:1901292] Also known as: nucleoside triphosphate breakdown, nucleoside triphosphate catabolism, nucleoside triphosphate degradation Subtypes: purine nucleoside triphosphate catabolic process [GO:0009146], GO:0009149, ribonucleoside triphosphate catabolic process [GO:0009203], deoxyribonucleoside triphosphate catabolic process [GO:0009204]